{
  "term_id": "GO:0016887",
  "gene_name": "Mitochondrial disaggregase",
  "gene_symbol": "CLPB",
  "gene": "UniProtKB:Q9H078",
  "term_label": "ATP hydrolysis activity"
}